{
  "gene_name": "Thymosin beta-10",
  "gene_symbol": "TMSB10",
  "gene": "UniProtKB:P63313",
  "term_id": "UNKNOWN:0003",
  "term_label": "Unknown cellular component"
}